{
  "gene_name": "Glycylpeptide N-tetradecanoyltransferase 2",
  "term_label": "protein localization to membrane",
  "gene": "UniProtKB:O60551",
  "term_id": "GO:0072657",
  "gene_symbol": "NMT2"
}